sarcosine catabolic process [GO:1901053] (biological process) References: PMID:17951379 Sources: GOC:TermGenie, GOC:yaf Definition: The chemical reactions and pathways resulting in the breakdown of sarcosine. Also known as: sarcosine breakdown, sarcosine catabolism, sarcosine degradation Relationships: is a type of GO:0042219; is a type of non-proteinogenic amino acid catabolic process [GO:0170044]; is a type of sarcosine metabolic process [GO:1901052]; is a type of GO:1901606